positive regulation of membrane depolarization during AV node cell action potential [GO:1905029] (biological process) References: PMID:19726871 Sources: GOC:BHF, GOC:BHF_miRNA, GOC:TermGenie, GOC:mtg_cardiac_conduct_nov11, GOC:rph Relationships: is a type of positive regulation of membrane depolarization during cardiac muscle cell action potential [GO:1900827]; is_a GO:1905027; positively regulates membrane depolarization during AV node cell action potential [GO:0086045] Also known as: positive regulation of membrane depolarization during AV node cardiac muscle cell action potential, positive regulation of membrane depolarization during atrioventricular node cardiac muscle cell action potential, up regulation of membrane depolarization during AV node cardiac muscle cell action potential, up regulation of membrane depolarization during AV node cell action potential, up regulation of membrane depolarization during atrioventricular node cardiac muscle cell action potential, up-regulation of membrane depolarization during AV node cardiac muscle cell action potential, up-regulation of membrane depolarization during AV node cell action potential, up-regulation of membrane depolarization during atrioventricular node cardiac muscle cell action potential, upregulation of membrane depolarization during AV node cardiac muscle cell action potential, upregulation of membrane depolarization during AV node cell action potential, upregulation of membrane depolarization during atrioventricular node cardiac muscle cell action potential, activation of membrane depolarization during AV node cardiac muscle cell action potential, activation of membrane depolarization during AV node cell action potential, activation of membrane depolarization during atrioventricular node cardiac muscle cell action potential Definition: Any process that activates or increases the frequency, rate or extent of membrane depolarization during AV node cell action potential.